{
  "gene_name": "SLIT and NTRK-like protein 1",
  "gene": "UniProtKB:Q96PX8",
  "gene_symbol": "SLITRK1",
  "term_id": "GO:0098839",
  "term_label": "postsynaptic density membrane"
}